{
  "gene_name": "Transcription initiation factor TFIID subunit 2",
  "gene": "UniProtKB:Q6P1X5",
  "term_id": "GO:0003682",
  "gene_symbol": "TAF2",
  "term_label": "chromatin binding"
}